{
  "term_label": "protein targeting to vacuole",
  "gene_symbol": "VPS37C",
  "term_id": "GO:0006623",
  "gene_name": "Vacuolar protein sorting-associated protein 37C",
  "gene": "UniProtKB:A5D8V6"
}